{
  "gene_symbol": "LLGL2",
  "term_id": "GO:0045159",
  "gene_name": "LLGL scribble cell polarity complex component 2",
  "gene": "UniProtKB:Q6P1M3",
  "term_label": "myosin II binding"
}